regulation of snoRNA processing [GO:1902796] (biological process) Definition: Any process that modulates the frequency, rate or extent of snoRNA processing. Relationships: is a type of regulation of gene expression [GO:0010468]; is a type of regulation of snoRNA metabolic process [GO:1903323]; regulates sno(s)RNA processing [GO:0043144] Subtypes: GO:1902797, positive regulation of snoRNA processing [GO:1902798] References: PMID:24210919 Sources: GOC:TermGenie, GO_REF:0000058